{
  "gene_name": "Synaptotagmin-11",
  "term_label": "exocytic vesicle",
  "gene": "UniProtKB:Q9BT88",
  "gene_symbol": "SYT11",
  "term_id": "GO:0070382"
}